{
  "gene_name": "Olfactory receptor 1A2",
  "gene": "UniProtKB:Q9Y585",
  "term_label": "plasma membrane",
  "gene_symbol": "OR1A2",
  "term_id": "GO:0005886"
}